{
  "gene_name": "Solute carrier organic anion transporter family member 3A1",
  "term_label": "Unknown molecular function",
  "term_id": "UNKNOWN:0001",
  "gene_symbol": "SLCO3A1",
  "gene": "UniProtKB:Q9UIG8"
}